{
  "gene_symbol": "TM4SF5",
  "term_label": "Unknown biological process",
  "gene_name": "Transmembrane 4 L6 family member 5",
  "term_id": "UNKNOWN:0002",
  "gene": "UniProtKB:O14894"
}